{
  "gene_name": "Transient receptor potential cation channel subfamily M member 5",
  "term_label": "metal ion transport",
  "gene": "UniProtKB:Q9NZQ8",
  "gene_symbol": "TRPM5",
  "term_id": "GO:0030001"
}